corneal epithelial cell differentiation [GO:0160122] (biological process) Relationships: is a type of epithelial cell differentiation [GO:0030855] Definition: The process in which a relatively unspecialized cell acquires specialized features of an corneal epithelial cell, any of the cells making up an corneal epithelium. References: PMID:32697979, PMID:33414365